4-hydroxyphenylacetate catabolic process [GO:1901023] (biological process) Definition: The chemical reactions and pathways resulting in the breakdown of 4-hydroxyphenylacetate. Also known as: 4-hydroxyphenylacetate breakdown, 4-hydroxyphenylacetate catabolism, 4-hydroxyphenylacetate degradation Relationships: is a type of GO:0019336; is a type of monocarboxylic acid catabolic process [GO:0072329]; is a type of GO:1901022 References: PMID:8550403 Sources: GOC:TermGenie, GOC:yaf